{
  "gene_symbol": "CPB2",
  "gene": "UniProtKB:Q96IY4",
  "term_label": "metallocarboxypeptidase activity",
  "gene_name": "Carboxypeptidase B2",
  "term_id": "GO:0004181"
}